{
  "gene_name": "Uncharacterized protein",
  "term_id": "UNKNOWN:0001",
  "term_label": "Unknown molecular function",
  "gene_symbol": "LOC122319696",
  "gene": "UniProtKB:A0A590UK24"
}